acylagmatine amidase activity [GO:0047618] (molecular function) Also known as: acylagmatine amidohydrolase activity, acylagmatine deacylase activity, benzoylagmatine amidohydrolase activity Sources: EC:3.5.1.40, RHEA:15065 Relationships: is a type of hydrolase activity, acting on carbon-nitrogen (but not peptide) bonds, in linear amides [GO:0016811] Definition: Catalysis of the reaction: N(4)-benzoylagmatine + H2O = agmatine + benzoate.